{
  "term_label": "T cell costimulation",
  "gene_symbol": "CD5",
  "term_id": "GO:0031295",
  "gene_name": "T-cell surface glycoprotein CD5",
  "gene": "UniProtKB:P06127"
}